{
  "term_id": "UNKNOWN:0003",
  "gene_name": "Olfactory receptor 11H6",
  "gene": "UniProtKB:Q8NGC7",
  "gene_symbol": "OR11H6",
  "term_label": "Unknown cellular component"
}